{
  "gene_name": "Rhotekin",
  "term_id": "GO:0005095",
  "term_label": "GTPase inhibitor activity",
  "gene": "UniProtKB:Q9BST9",
  "gene_symbol": "RTKN"
}